{
  "gene_symbol": "RND3",
  "term_id": "GO:0019901",
  "gene": "UniProtKB:P61587",
  "gene_name": "Rho-related GTP-binding protein RhoE",
  "term_label": "protein kinase binding"
}